{
  "gene_symbol": "CRPPA",
  "gene_name": "D-ribitol-5-phosphate cytidylyltransferase",
  "term_label": "cytosol",
  "gene": "UniProtKB:A4D126",
  "term_id": "GO:0005829"
}